{
  "gene": "UniProtKB:Q8TCT7",
  "gene_name": "Signal peptide peptidase-like 2B",
  "term_id": "GO:0033619",
  "term_label": "membrane protein proteolysis",
  "gene_symbol": "SPPL2B"
}